{
  "term_label": "G protein-coupled receptor signaling pathway",
  "term_id": "GO:0007186",
  "gene_symbol": "TAAR1",
  "gene_name": "Trace amine-associated receptor 1",
  "gene": "UniProtKB:Q96RJ0"
}